{
  "gene_name": "Phospholipid transfer protein",
  "term_id": "GO:0015914",
  "term_label": "phospholipid transport",
  "gene": "UniProtKB:P55058",
  "gene_symbol": "PLTP"
}